glutathione transport [GO:0034635] (biological process) Definition: The directed movement of glutathione, the tripeptide glutamylcysteinylglycine, into, out of or within a cell, or between cells, by means of some agent such as a transporter or pore. Subtypes: glutathione transmembrane transport [GO:0034775] Sources: GOC:mah Relationships: is a type of organic anion transport [GO:0015711]; is a type of GO:0042939; is a type of GO:0072337; is a type of sulfur compound transport [GO:0072348]